positive regulation of atrichoblast fate specification [GO:0010059] (biological process) Definition: Any process that induces or promotes atrichoblast fate specification. Sources: GOC:tb Also known as: up regulation of atrichoblast fate, up-regulation of atrichoblast fate, upregulation of atrichoblast fate, activation of atrichoblast fate, stimulation of atrichoblast fate Relationships: is a type of regulation of atrichoblast fate specification [GO:0010058]; is a type of positive regulation of cell fate specification [GO:0042660]; is a type of positive regulation of plant epidermal cell differentiation [GO:1903890]; positively regulates atrichoblast fate specification [GO:0010056]